{
  "term_id": "UNKNOWN:0001",
  "gene_symbol": "FBLN1",
  "term_label": "Unknown molecular function",
  "gene": "UniProtKB:P23142",
  "gene_name": "Fibulin-1"
}